dGTP diphosphatase activity [GO:0036217] (molecular function) Also known as: 2'-deoxyguanosine 5'-triphosphate diphosphohydrolase, dGTP pyrophosphatase activity Definition: Catalysis of the reaction: dGTP + H2O = dGMP + H+ + diphosphate. Relationships: is a type of nucleoside triphosphate diphosphatase activity [GO:0047429] References: PMID:17090528, PMID:22531138 Sources: GOC:dgf, RHEA:28362